{
  "term_id": "GO:0051382",
  "term_label": "kinetochore assembly",
  "gene": "UniProtKB:P0DPK2",
  "gene_name": "Histone H3.Y",
  "gene_symbol": "H3Y1"
}